{
  "gene": "UniProtKB:P83436",
  "term_label": "retrograde vesicle-mediated transport, Golgi to endoplasmic reticulum",
  "gene_name": "Conserved oligomeric Golgi complex subunit 7",
  "gene_symbol": "COG7",
  "term_id": "GO:0006890"
}